{
  "gene_name": "Zinc finger FYVE domain-containing protein 21",
  "gene": "UniProtKB:Q9BQ24",
  "term_label": "Unknown biological process",
  "term_id": "UNKNOWN:0002",
  "gene_symbol": "ZFYVE21"
}